{
  "gene": "UniProtKB:P13995",
  "term_id": "GO:0004488",
  "gene_symbol": "MTHFD2",
  "gene_name": "Bifunctional methylenetetrahydrofolate dehydrogenase_cyclohydrolase, mitochondrial",
  "term_label": "methylenetetrahydrofolate dehydrogenase (NADP+) activity"
}